glutamate-prephenate aminotransferase activity [GO:0033854] (MF) Relationships: is a type of transaminase activity [GO:0008483] Sources: EC:2.6.1.79, RHEA:22880 Definition: Catalysis of the reaction: 2-oxoglutarate + L-arogenate = L-glutamate + prephenate. Also known as: prephenate transaminase activity, L-arogenate:2-oxoglutarate aminotransferase activity, L-glutamate:prephenate aminotransferase activity, PAT